regulation of plasma membrane organization [GO:1903729] (biological process) Also known as: regulation of plasma membrane organisation, regulation of plasma membrane organization and biogenesis References: PMID:24514900 Sources: GOC:TermGenie, GO_REF:0000058 Subtypes: regulation of fusion of sperm to egg plasma membrane [GO:0043012], GO:1903525, regulation of plasma membrane raft polarization [GO:1903906], regulation of plasma membrane repair [GO:1905684], GO:1905780 Relationships: is a type of regulation of cellular component organization [GO:0051128]; regulates plasma membrane organization [GO:0007009] Definition: Any process that modulates the frequency, rate or extent of plasma membrane organization.